phagophore assembly site membrane [GO:0034045] (cellular component) References: PMID:16874040, PMID:17382324 Sources: GOC:mah, GOC:rph Definition: A cellular membrane associated with the phagophore assembly site. Relationships: is a type of membrane [GO:0016020]; is part of GO:0000407 Also known as: PAS membrane, pre-autophagosomal structure membrane, isolation membrane, phagophore